{
  "gene_symbol": "GRIN3A",
  "gene": "UniProtKB:Q8TCU5",
  "gene_name": "Glutamate receptor ionotropic, NMDA 3A",
  "term_id": "GO:0035249",
  "term_label": "synaptic transmission, glutamatergic"
}